{
  "gene_name": "ADP-ribosylation factor-like protein 4C",
  "term_label": "endocytic recycling",
  "gene_symbol": "ARL4C",
  "term_id": "GO:0032456",
  "gene": "UniProtKB:P56559"
}